positive regulation of hexokinase activity [GO:1903301] (biological process) Relationships: is a type of positive regulation of kinase activity [GO:0033674]; positively regulates hexokinase activity [GO:0004396] References: PMID:15804508 Sources: GOC:TermGenie, GOC:mr, GO_REF:0000059 Also known as: positive regulation of ATP-dependent hexokinase activity, positive regulation of ATP:D-hexose 6-phosphotransferase activity, positive regulation of glucose ATP phosphotransferase activity, positive regulation of hexokinase (phosphorylating), positive regulation of hexokinase type IV glucokinase activity, up regulation of ATP-dependent hexokinase activity, up regulation of ATP:D-hexose 6-phosphotransferase activity, up regulation of glucose ATP phosphotransferase activity, up regulation of hexokinase (phosphorylating), up regulation of hexokinase activity, up regulation of hexokinase type IV glucokinase activity, up-regulation of ATP-dependent hexokinase activity, up-regulation of ATP:D-hexose 6-phosphotransferase activity, up-regulation of glucose ATP phosphotransferase activity, up-regulation of hexokinase (phosphorylating), up-regulation of hexokinase activity, up-regulation of hexokinase type IV glucokinase activity, upregulation of ATP-dependent hexokinase activity, upregulation of ATP:D-hexose 6-phosphotransferase activity, upregulation of glucose ATP phosphotransferase activity, upregulation of hexokinase (phosphorylating), upregulation of hexokinase activity, upregulation of hexokinase type IV glucokinase activity, activation of ATP-dependent hexokinase activity, activation of ATP:D-hexose 6-phosphotransferase activity, activation of glucose ATP phosphotransferase activity, activation of hexokinase (phosphorylating), activation of hexokinase activity, activation of hexokinase type I activity, activation of hexokinase type II activity, activation of hexokinase type III activity, activation of hexokinase type IV (glucokinase) activity, activation of hexokinase type IV glucokinase activity, positive regulation of hexokinase type I activity, positive regulation of hexokinase type II activity, positive regulation of hexokinase type III activity, positive regulation of hexokinase type IV (glucokinase) activity, up regulation of hexokinase type I activity, up regulation of hexokinase type II activity, up regulation of hexokinase type III activity, up regulation of hexokinase type IV (glucokinase) activity, up-regulation of hexokinase type I activity, up-regulation of hexokinase type II activity, up-regulation of hexokinase type III activity, up-regulation of hexokinase type IV (glucokinase) activity, upregulation of hexokinase type I activity, upregulation of hexokinase type II activity, upregulation of hexokinase type III activity, upregulation of hexokinase type IV (glucokinase) activity, activation of hexokinase D, activation of hexokinase type IV, positive regulation of hexokinase D, positive regulation of hexokinase type IV, up regulation of hexokinase D, up regulation of hexokinase type IV, up-regulation of hexokinase D, up-regulation of hexokinase type IV, upregulation of hexokinase D, upregulation of hexokinase type IV Definition: Any process that activates or increases the frequency, rate or extent of hexokinase activity.